{
  "gene_symbol": "H2AC17",
  "gene_name": "Histone H2A type 1",
  "term_label": "heterochromatin formation",
  "term_id": "GO:0031507",
  "gene": "UniProtKB:P0C0S8"
}